{
  "gene": "UniProtKB:Q03828",
  "term_label": "nucleus",
  "term_id": "GO:0005634",
  "gene_symbol": "EVX2",
  "gene_name": "Homeobox even-skipped homolog protein 2"
}